interleukin-21 receptor activity [GO:0001532] (molecular function) Sources: GOC:jl, GOC:signaling Definition: Combining with interleukin-21 and transmitting the signal from one side of the membrane to the other to initiate a change in cell activity. Relationships: is a type of cytokine receptor activity [GO:0004896]; is part of interleukin-21-mediated signaling pathway [GO:0038114]; has part GO:0019977 Also known as: IL-21 receptor activity, IL-21R